{
  "term_label": "Unknown cellular component",
  "gene": "UniProtKB:A0A075B6Z2",
  "term_id": "UNKNOWN:0003",
  "gene_name": "T cell receptor alpha joining 56 (Fragment)",
  "gene_symbol": "TRAJ56"
}